{
  "gene_symbol": "PRPSAP1",
  "term_id": "GO:0006164",
  "gene_name": "Phosphoribosyl pyrophosphate synthase-associated protein 1",
  "gene": "UniProtKB:Q14558",
  "term_label": "purine nucleotide biosynthetic process"
}